{
  "term_label": "plasma membrane",
  "gene_symbol": "ENTPD2",
  "gene": "UniProtKB:Q9Y5L3",
  "gene_name": "Ectonucleoside triphosphate diphosphohydrolase 2",
  "term_id": "GO:0005886"
}